{
  "term_label": "Golgi organization",
  "gene": "UniProtKB:Q9NYA3",
  "gene_symbol": "GOLGA6A",
  "term_id": "GO:0007030",
  "gene_name": "Golgin subfamily A member 6A"
}